urate catabolic process [GO:0019628] (biological process) Definition: The chemical reactions and pathways resulting in the breakdown of urate, the anion of uric acid, 2,6,8-trioxypurine. Sources: ISBN:0198506732 Relationships: is a type of small molecule catabolic process [GO:0044282]; is a type of urate metabolic process [GO:0046415]; is a type of purine-containing compound catabolic process [GO:0072523] Also known as: urate breakdown, urate catabolism, urate degradation, uric acid catabolic process